{
  "gene_name": "Putative protein FAM86C2P",
  "gene": "UniProtKB:A6NEL3",
  "term_id": "UNKNOWN:0002",
  "term_label": "Unknown biological process",
  "gene_symbol": "FAM86C2P"
}